{
  "gene_name": "Sodium_potassium_calcium exchanger 1",
  "term_label": "plasma membrane",
  "term_id": "GO:0005886",
  "gene_symbol": "SLC24A1",
  "gene": "UniProtKB:O60721"
}